{
  "term_label": "cytosol",
  "gene_name": "Rho GTPase-activating protein 10",
  "gene": "UniProtKB:A1A4S6",
  "gene_symbol": "ARHGAP10",
  "term_id": "GO:0005829"
}